regulation of synaptonemal complex assembly [GO:0090173] (biological process) Definition: Any process that modulates the frequency, rate or extent of synaptonemal complex assembly. Synaptonemal complex assembly is the cell cycle process in which the synaptonemal complex, a structure that holds paired chromosomes together during prophase I of meiosis and that promotes genetic recombination, is formed. Relationships: is a type of regulation of cell cycle process [GO:0010564]; is a type of regulation of chromosome organization [GO:0033044]; is a type of regulation of cellular component biogenesis [GO:0044087]; is a type of regulation of reproductive process [GO:2000241]; regulates GO:0007130 Subtypes: positive regulation of synaptonemal complex assembly [GO:1905088] Sources: GOC:ascb_2009, GOC:dph, GOC:tb